{
  "gene_name": "Transmembrane and coiled-coil domains protein 1",
  "gene": "UniProtKB:O94876",
  "gene_symbol": "TMCC1",
  "term_id": "GO:0140285",
  "term_label": "endosome fission"
}